{
  "gene_name": "Rho GTPase-activating protein 22",
  "gene": "UniProtKB:Q7Z5H3",
  "term_label": "negative regulation of small GTPase mediated signal transduction",
  "term_id": "GO:0051058",
  "gene_symbol": "ARHGAP22"
}